{
  "gene_name": "SWI_SNF-related matrix-associated actin-dependent regulator of chromatin subfamily A containing DEAD_H box 1",
  "term_label": "heterochromatin formation",
  "term_id": "GO:0031507",
  "gene": "UniProtKB:Q9H4L7",
  "gene_symbol": "SMARCAD1"
}